{
  "gene_symbol": "ABHD10",
  "gene_name": "Palmitoyl-protein thioesterase ABHD10, mitochondrial",
  "gene": "UniProtKB:Q9NUJ1",
  "term_id": "GO:0008474",
  "term_label": "palmitoyl-(protein) hydrolase activity"
}